positive regulation of cell-cell adhesion mediated by integrin [GO:0033634] (biological process) Definition: Any process that activates or increases the frequency, rate, or extent of cell-cell adhesion mediated by integrin. Sources: GOC:add Also known as: positive regulation of cell-cell adhesion mediated by integrin complex Relationships: is a type of GO:0022409; is a type of positive regulation of cell adhesion mediated by integrin [GO:0033630]; is a type of GO:0033632; positively regulates cell-cell adhesion mediated by integrin [GO:0033631]